{
  "gene_name": "Zinc phosphodiesterase ELAC protein 1",
  "term_id": "GO:0005634",
  "term_label": "nucleus",
  "gene_symbol": "ELAC1",
  "gene": "UniProtKB:Q9H777"
}